{
  "gene_name": "Coiled-coil domain-containing protein 38",
  "gene_symbol": "CCDC38",
  "gene": "UniProtKB:Q502W7",
  "term_label": "Unknown molecular function",
  "term_id": "UNKNOWN:0001"
}